{
  "gene_name": "Checkpoint protein HUS1B",
  "term_label": "double-strand break repair via homologous recombination",
  "gene_symbol": "HUS1B",
  "term_id": "GO:0000724",
  "gene": "UniProtKB:Q8NHY5"
}